{
  "gene_name": "DnaJ homolog subfamily B member 6",
  "term_label": "cytoplasm",
  "term_id": "GO:0005737",
  "gene_symbol": "DNAJB6",
  "gene": "UniProtKB:O75190"
}